sister chromatid biorientation [GO:0031134] (biological process) Definition: The cell cycle process in which sister chromatids establish stable attachments to microtubules emanating from opposite spindle poles. References: PMID:15309047 Also known as: chromosome biorientation, sister kinetochore biorientation Relationships: is a type of GO:0008608; is part of sister chromatid segregation [GO:0000819] Subtypes: mitotic sister chromatid biorientation [GO:1990758]